{
  "gene_name": "Immunoglobulin heavy variable 1-2",
  "term_label": "antigen binding",
  "gene": "UniProtKB:P23083",
  "term_id": "GO:0003823",
  "gene_symbol": "IGHV1-2"
}